{
  "gene_name": "Putative homeobox protein Meis3-like 2",
  "gene": "UniProtKB:A8K0S8",
  "gene_symbol": "MEIS3P2",
  "term_label": "positive regulation of cell population proliferation",
  "term_id": "GO:0008284"
}